{
  "term_label": "actin polymerization-dependent cell motility",
  "gene_name": "Protein enabled homolog",
  "gene_symbol": "ENAH",
  "gene": "UniProtKB:Q8N8S7",
  "term_id": "GO:0070358"
}